{
  "gene_symbol": "DNAJC28",
  "gene": "UniProtKB:Q9NX36",
  "term_id": "GO:0001659",
  "gene_name": "DnaJ homolog subfamily C member 28",
  "term_label": "temperature homeostasis"
}